{
  "gene_symbol": "CCNF",
  "gene": "UniProtKB:P41002",
  "term_label": "nucleus",
  "gene_name": "Cyclin-F",
  "term_id": "GO:0005634"
}